{
  "term_label": "cardiolipin biosynthetic process",
  "gene_symbol": "CRLS1",
  "gene_name": "Cardiolipin synthase (CMP-forming)",
  "term_id": "GO:0032049",
  "gene": "UniProtKB:Q9UJA2"
}